ATP-binding cassette (ABC) transporter complex, integrated substrate binding [GO:0055051] (cellular component) Sources: GOC:mlg, GOC:mtg_sensu Definition: A complex for the transport of metabolites out of the cell, consisting of 4 domains: two ATP-binding domains and two membrane spanning domains. In some cases, all 4 domains are contained on 1 polypeptide, while in others one ATP-binding domain and one membrane spanning domain are together on one polypeptide in what is called a half transporter. Two half-transporters come together to form a functional transporter. Transport of the substrate across the membrane is driven by the hydrolysis of ATP. Relationships: is a type of ATP-binding cassette (ABC) transporter complex [GO:0043190]